{
  "gene_name": "Cholecystokinin receptor type A",
  "term_id": "GO:0046883",
  "term_label": "regulation of hormone secretion",
  "gene_symbol": "CCKAR",
  "gene": "UniProtKB:P32238"
}